regulation of peripheral tolerance induction [GO:0002658] (biological process) Sources: GOC:add Definition: Any process that modulates the frequency, rate, or extent of peripheral tolerance induction. Subtypes: negative regulation of peripheral tolerance induction [GO:0002659], positive regulation of peripheral tolerance induction [GO:0002660], regulation of tolerance induction to tumor cell [GO:0002843], regulation of peripheral T cell tolerance induction [GO:0002849], regulation of peripheral B cell deletion [GO:0002908], regulation of peripheral B cell anergy [GO:0002917] Relationships: is a type of regulation of tolerance induction dependent upon immune response [GO:0002652]; regulates GO:0002465